{
  "term_id": "UNKNOWN:0002",
  "gene_name": "Adiponectin",
  "term_label": "Unknown biological process",
  "gene_symbol": "ADIPOQ",
  "gene": "UniProtKB:Q15848"
}